{
  "term_id": "GO:0008568",
  "term_label": "microtubule severing ATPase activity",
  "gene": "UniProtKB:A6NCM1",
  "gene_symbol": "IQCA1L",
  "gene_name": "IQ and AAA domain-containing protein 1-like"
}